{
  "gene_symbol": "Q6ZTK2",
  "gene": "UniProtKB:Q6ZTK2",
  "term_id": "UNKNOWN:0002",
  "gene_name": "Putative uncharacterized protein LOC400499",
  "term_label": "Unknown biological process"
}